{
  "term_id": "GO:0007030",
  "term_label": "Golgi organization",
  "gene": "UniProtKB:Q08379",
  "gene_name": "Golgin subfamily A member 2",
  "gene_symbol": "GOLGA2"
}